TRAF2-GSTP1 complex [GO:0097057] (cellular component) Relationships: is a type of protein-containing complex [GO:0032991] Definition: A protein complex comprising tumor necrosis factor (TNF) receptor-associated factor 2 (TRAF2) and glutathione S-transferase pi 1 (GSTP1). This complex is thought to disrupt the TNF signaling cascade, thus down-regulating inflammatory responses. References: PMID:16636664 Sources: GOC:BHF